{
  "gene": "UniProtKB:P10720",
  "gene_name": "Platelet factor 4 variant",
  "gene_symbol": "PF4V1",
  "term_id": "GO:0005615",
  "term_label": "extracellular space"
}